{
  "term_label": "fertilization",
  "gene": "UniProtKB:A6NMN3",
  "gene_symbol": "FAM170B",
  "term_id": "GO:0009566",
  "gene_name": "Protein FAM170B"
}